negative regulation of lipoprotein transport [GO:0140076] (biological process) Relationships: is a type of negative regulation of protein transport [GO:0051224]; is a type of regulation of lipoprotein transport [GO:0140075]; negatively regulates lipoprotein transport [GO:0042953] Definition: Any process that stops, prevents or reduces the frequency, rate or extent of lipoprotein transport. References: PMID:26501192 Sources: GOC:BHF, GOC:BHF_miRNA, GOC:RPH